{
  "gene_name": "X-ray radiation resistance-associated protein 1",
  "term_label": "nucleus",
  "gene_symbol": "XRRA1",
  "gene": "UniProtKB:Q6P2D8",
  "term_id": "GO:0005634"
}